{
  "term_id": "GO:0016913",
  "gene": "UniProtKB:P01215",
  "gene_symbol": "CGA",
  "gene_name": "Glycoprotein hormones alpha chain",
  "term_label": "follicle-stimulating hormone activity"
}